{
  "gene": "UniProtKB:Q8TF32",
  "term_id": "UNKNOWN:0003",
  "gene_symbol": "ZNF431",
  "term_label": "Unknown cellular component",
  "gene_name": "Zinc finger protein 431"
}